{
  "gene_symbol": "AIRE",
  "term_id": "GO:0042393",
  "gene": "UniProtKB:O43918",
  "term_label": "histone binding",
  "gene_name": "Autoimmune regulator"
}